forebrain neuroblast division [GO:0021873] (biological process) Definition: The division of a neuroblast located in the forebrain. Neuroblast division gives rise to at least another neuroblast. Sources: GOC:cls, GOC:dgh, GOC:dph, GOC:jid, GO_REF:0000021 Subtypes: GO:0021847, GO:0022017 Relationships: is a type of neuroblast division [GO:0055057]; is part of forebrain generation of neurons [GO:0021872]